{
  "term_label": "Unknown cellular component",
  "gene": "UniProtKB:Q9NS84",
  "gene_name": "Carbohydrate sulfotransferase 7",
  "term_id": "UNKNOWN:0003",
  "gene_symbol": "CHST7"
}